renal sodium excretion [GO:0035812] (biological process) Definition: The elimination of sodium ions from peritubular capillaries (or surrounding hemolymph in invertebrates) into the renal tubules to be incorporated subsequently into the urine. References: PMID:25287933 Sources: GOC:mtg_25march11, GOC:yaf Regulation: regulated by regulation of renal sodium excretion [GO:0035813]; negatively regulated by GO:0035814; positively regulated by positive regulation of renal sodium excretion [GO:0035815] Relationships: is a type of renal tubular secretion [GO:0097254]; is part of sodium ion homeostasis [GO:0055078]